{
  "gene": "UniProtKB:P49755",
  "gene_name": "Transmembrane emp24 domain-containing protein 10",
  "gene_symbol": "TMED10",
  "term_label": "COPII-coated ER to Golgi transport vesicle",
  "term_id": "GO:0030134"
}